{
  "term_id": "GO:0005737",
  "gene": "UniProtKB:O43781",
  "term_label": "cytoplasm",
  "gene_symbol": "DYRK3",
  "gene_name": "Dual specificity tyrosine-phosphorylation-regulated kinase 3"
}